{
  "term_id": "GO:0000995",
  "gene": "UniProtKB:Q92994",
  "gene_name": "Transcription factor IIIB 90 kDa subunit",
  "gene_symbol": "BRF1",
  "term_label": "RNA polymerase III general transcription initiation factor activity"
}